{
  "term_label": "chromatin binding",
  "gene_name": "Putative Dresden prostate carcinoma protein 2",
  "gene": "UniProtKB:Q86SG4",
  "term_id": "GO:0003682",
  "gene_symbol": "HMGN2P46"
}